{
  "term_label": "Unknown cellular component",
  "gene_symbol": "SPMIP10",
  "gene": "UniProtKB:Q6ZNM6",
  "term_id": "UNKNOWN:0003",
  "gene_name": "Testis-expressed protein 43"
}